{
  "gene_name": "Myelodysplastic syndrome 2 translocation-associated protein",
  "gene": "UniProtKB:Q8NDY4",
  "term_label": "Unknown biological process",
  "gene_symbol": "MDS2",
  "term_id": "UNKNOWN:0002"
}